{
  "gene_name": "NADPH oxidase 1",
  "gene_symbol": "NOX1",
  "term_id": "GO:0043020",
  "gene": "UniProtKB:Q9Y5S8",
  "term_label": "NADPH oxidase complex"
}